{
  "term_id": "GO:0004523",
  "gene_symbol": "RNASEH1",
  "gene_name": "Ribonuclease H1",
  "term_label": "RNA-DNA hybrid ribonuclease activity",
  "gene": "UniProtKB:O60930"
}